{
  "gene": "UniProtKB:Q9NXG2",
  "gene_name": "THUMP domain-containing protein 1",
  "gene_symbol": "THUMPD1",
  "term_label": "RNA binding",
  "term_id": "GO:0003723"
}